{
  "gene": "UniProtKB:Q7L2H7",
  "term_label": "cytoplasmic translational initiation",
  "gene_symbol": "EIF3M",
  "gene_name": "Eukaryotic translation initiation factor 3 subunit M",
  "term_id": "GO:0002183"
}